{
  "gene_symbol": "HCAR3",
  "term_id": "GO:0005886",
  "term_label": "plasma membrane",
  "gene": "UniProtKB:P49019",
  "gene_name": "Hydroxycarboxylic acid receptor 3"
}